{
  "gene_symbol": "DLST",
  "gene_name": "Dihydrolipoyllysine-residue succinyltransferase component of 2-oxoglutarate dehydrogenase complex, mitochondrial",
  "term_label": "dihydrolipoyllysine-residue succinyltransferase activity",
  "term_id": "GO:0004149",
  "gene": "UniProtKB:P36957"
}